{
  "term_label": "protein retention in ER lumen",
  "term_id": "GO:0006621",
  "gene": "UniProtKB:O43731",
  "gene_name": "ER lumen protein-retaining receptor 3",
  "gene_symbol": "KDELR3"
}